antennal joint morphogenesis [GO:0048801] (biological process) Definition: The process in which the anatomical structures of the antennal joint are generated and organized. Sources: GOC:jid Relationships: is a type of post-embryonic animal morphogenesis [GO:0009886]; is part of antennal joint development [GO:0048098]; is part of GO:0048800